{
  "term_id": "GO:0071723",
  "term_label": "lipopeptide binding",
  "gene_name": "T-cell surface glycoprotein CD1b",
  "gene_symbol": "CD1B",
  "gene": "UniProtKB:P29016"
}